{
  "gene": "UniProtKB:Q96TA1",
  "term_id": "UNKNOWN:0002",
  "gene_name": "Protein Niban 2",
  "term_label": "Unknown biological process",
  "gene_symbol": "NIBAN2"
}